{
  "gene_symbol": "LRRC75A",
  "term_id": "GO:1990756",
  "gene_name": "Leucine-rich repeat-containing protein 75A",
  "gene": "UniProtKB:Q8NAA5",
  "term_label": "ubiquitin-like ligase-substrate adaptor activity"
}